{
  "term_id": "UNKNOWN:0002",
  "gene_symbol": "FAM133A",
  "gene": "UniProtKB:Q8N9E0",
  "gene_name": "Protein FAM133A",
  "term_label": "Unknown biological process"
}